{
  "gene_symbol": "SEC11B",
  "gene": "UniProtKB:P0C7V7",
  "gene_name": "Putative signal peptidase complex catalytic subunit SEC11B",
  "term_label": "signal peptidase complex",
  "term_id": "GO:0005787"
}